{
  "gene": "UniProtKB:Q9NT62",
  "term_id": "GO:0000407",
  "term_label": "phagophore assembly site",
  "gene_name": "Ubiquitin-like-conjugating enzyme ATG3",
  "gene_symbol": "ATG3"
}